CD4-positive, CD25-positive, alpha-beta regulatory T cell lineage commitment [GO:0002362] (biological process) References: PMID:15207821 Sources: GOC:add Relationships: is a type of GO:0043373; is part of CD4-positive, CD25-positive, alpha-beta regulatory T cell differentiation [GO:0002361] Also known as: CD4-positive, CD25-positive, alpha-beta regulatory T lymphocyte lineage commitment, CD4-positive, CD25-positive, alpha-beta regulatory T-cell lineage commitment, CD4-positive, CD25-positive, alpha-beta regulatory T-lymphocyte lineage commitment Definition: The process in which a CD4-positive, alpha-beta T cell becomes committed to becoming a CD4-positive, CD25-positive, alpha-beta regulatory T cell.